{
  "term_id": "UNKNOWN:0002",
  "term_label": "Unknown biological process",
  "gene_symbol": "H1-10-AS1",
  "gene_name": "Putative uncharacterized protein H1-10-AS1",
  "gene": "UniProtKB:Q4G0G2"
}